{
  "term_id": "GO:0004467",
  "gene_symbol": "ACSL3",
  "term_label": "long-chain fatty acid-CoA ligase activity",
  "gene": "UniProtKB:O95573",
  "gene_name": "Fatty acid CoA ligase Acsl3"
}